positive regulation of endopeptidase activity [GO:0010950] (biological process) Subtypes: positive regulation of serine-type endopeptidase activity [GO:1900005], GO:1904685 Sources: GOC:dph, GOC:tb Definition: Any process that increases the frequency, rate or extent of endopeptidase activity, the endohydrolysis of peptide bonds within proteins. Relationships: is a type of GO:0010952; is a type of regulation of endopeptidase activity [GO:0052548]; positively regulates endopeptidase activity [GO:0004175]